{
  "gene_name": "Amyloid-beta precursor protein",
  "term_id": "GO:0005886",
  "gene_symbol": "APP",
  "term_label": "plasma membrane",
  "gene": "UniProtKB:P05067"
}